{
  "gene": "UniProtKB:Q5VYV0",
  "term_label": "RNA polymerase II cis-regulatory region sequence-specific DNA binding",
  "term_id": "GO:0000978",
  "gene_name": "Forkhead box protein B2",
  "gene_symbol": "FOXB2"
}